viral double stranded DNA replication via reverse transcription [GO:0039688] (biological process) Definition: A DNA replication process that uses viral RNA as a template for RNA-dependent DNA polymerases (e.g. reverse transcriptase) that synthesize the new strands. Relationships: is a type of GO:0039693; has part reverse transcription [GO:0001171]; has part DNA-templated viral transcription [GO:0039695] Sources: GOC:bf, GOC:jl, VZ:1938 Also known as: dsDNA replication via RNA intermediate, viral RNA-dependent DNA replication, RNA-dependent viral DNA replication